pole plasm mitochondrial srRNA localization [GO:0019097] (biological process) Also known as: establishment and maintenance of mitochondrial localization in pole plasm, oocyte pole plasm mitochondrial srRNA localization, pole plasm mitochondrial srRNA localisation Definition: Any process in which mitochondrial small ribosomal RNA is transported to, or maintained in, the oocyte pole plasm. An example of this is found in Drosophila melanogaster. Sources: ISBN:0879694238 Relationships: is a type of pole plasm mitochondrial rRNA localization [GO:0019095]